{
  "gene_symbol": "ESCO1",
  "gene_name": "N-acetyltransferase ESCO1",
  "gene": "UniProtKB:Q5FWF5",
  "term_label": "mitotic sister chromatid cohesion",
  "term_id": "GO:0007064"
}